specification of pronephric tubule identity [GO:0039005] (biological process) Sources: GOC:mtg_kidney_jan10 Definition: The process in which the tubules arranged along the proximal/distal axis of the pronephric nephron acquire their identity. Subtypes: GO:0039004, GO:0039010 Relationships: is a type of pattern specification involved in pronephros development [GO:0039017]; is a type of specification of nephron tubule identity [GO:0072081]; is part of pronephric nephron tubule morphogenesis [GO:0039008]